trans-feruloyl-CoA synthase activity [GO:0050563] (molecular function) Also known as: ferulate-CoA ligase activity, trans-ferulate:CoASH ligase (ATP-hydrolysing), trans-feruloyl-CoA synthetase activity Relationships: is a type of GO:0016405 References: PMID:22649270 Sources: EC:6.2.1.34 Definition: Catalysis of the reaction: ATP + CoA + trans-ferulate = (E)-feruloyl-CoA + ADP + phosphate. ADP + phosphate or AMP + diphosphate may be formed in this reaction.